regulation of miRNA catabolic process [GO:2000625] (biological process) Definition: Any process that modulates the frequency, rate or extent of miRNA catabolic process. Sources: GOC:dph Also known as: regulation of microRNA catabolic process Relationships: is a type of regulation of catabolic process [GO:0009894]; is a type of regulation of miRNA metabolic process [GO:2000628]; regulates GO:0010587 Subtypes: GO:2000626, positive regulation of miRNA catabolic process [GO:2000627]